{
  "gene_symbol": "VAX1",
  "gene_name": "Ventral anterior homeobox 1",
  "term_label": "central nervous system development",
  "term_id": "GO:0007417",
  "gene": "UniProtKB:Q5SQQ9"
}